{
  "term_id": "GO:0004364",
  "gene": "UniProtKB:Q9Y2Q3",
  "gene_symbol": "GSTK1",
  "term_label": "glutathione transferase activity",
  "gene_name": "Glutathione S-transferase kappa 1"
}